{
  "term_id": "GO:0004180",
  "gene_symbol": "NAALADL1",
  "gene": "UniProtKB:Q9UQQ1",
  "term_label": "carboxypeptidase activity",
  "gene_name": "Aminopeptidase NAALADL1"
}